{
  "gene_symbol": "WLS",
  "gene": "UniProtKB:Q5T9L3",
  "term_label": "endomembrane system",
  "gene_name": "Protein wntless homolog",
  "term_id": "GO:0012505"
}